{
  "term_label": "endothelin receptor activity",
  "gene_name": "Endothelin-1 receptor",
  "term_id": "GO:0004962",
  "gene_symbol": "EDNRA",
  "gene": "UniProtKB:P25101"
}